positive regulation of JNK cascade [GO:0046330] (biological process) Sources: GOC:bf Also known as: up regulation of JNK cascade, up-regulation of JNK cascade, upregulation of JNK cascade, activation of JNK cascade, stimulation of JNK cascade Definition: Any process that activates or increases the frequency, rate or extent of signal transduction mediated by the JNK cascade. Relationships: is a type of positive regulation of MAPK cascade [GO:0043410]; is a type of regulation of JNK cascade [GO:0046328]; positively regulates JNK cascade [GO:0007254]